{
  "term_label": "regulation of intracellular pH",
  "gene": "UniProtKB:Q9UBY0",
  "term_id": "GO:0051453",
  "gene_name": "Sodium_hydrogen exchanger 2",
  "gene_symbol": "SLC9A2"
}